{
  "term_id": "UNKNOWN:0001",
  "term_label": "Unknown molecular function",
  "gene_symbol": "BCL7C",
  "gene": "UniProtKB:Q8WUZ0",
  "gene_name": "B-cell CLL_lymphoma 7 protein family member C"
}